{
  "gene": "UniProtKB:Q969J3",
  "gene_name": "BLOC-1-related complex subunit 5",
  "term_label": "lysosome localization",
  "term_id": "GO:0032418",
  "gene_symbol": "BORCS5"
}